{
  "term_label": "intracellular protein localization",
  "gene": "UniProtKB:Q9P0V9",
  "term_id": "GO:0008104",
  "gene_symbol": "SEPTIN10",
  "gene_name": "Septin-10"
}